{
  "gene_symbol": "PLAAT5",
  "gene": "UniProtKB:Q96KN8",
  "term_id": "GO:0008970",
  "gene_name": "Phospholipase A and acyltransferase 5",
  "term_label": "phospholipase A1 activity"
}